{
  "term_label": "cytoplasm",
  "gene": "UniProtKB:P12429",
  "term_id": "GO:0005737",
  "gene_symbol": "ANXA3",
  "gene_name": "Annexin A3"
}